{
  "term_label": "DNA-binding transcription repressor activity, RNA polymerase II-specific",
  "term_id": "GO:0001227",
  "gene_name": "Insulinoma-associated protein 2",
  "gene": "UniProtKB:Q96T92",
  "gene_symbol": "INSM2"
}